{
  "term_id": "GO:0004725",
  "gene_name": "Tensin-2",
  "gene": "UniProtKB:Q63HR2",
  "gene_symbol": "TNS2",
  "term_label": "protein tyrosine phosphatase activity"
}